{
  "term_label": "membrane attack complex",
  "gene_symbol": "C8G",
  "term_id": "GO:0005579",
  "gene_name": "Complement component C8 gamma chain",
  "gene": "UniProtKB:P07360"
}